host cell projection [GO:0044157] (cellular component) Subtypes: host cell filopodium [GO:0044176], GO:0120026 Sources: GOC:rph Relationships: is a type of GO:0033643 Definition: A prolongation or process extending from a host cell, e.g. a flagellum or axon.